{
  "gene": "UniProtKB:O75081",
  "gene_symbol": "CBFA2T3",
  "term_label": "transcription corepressor activity",
  "gene_name": "Protein CBFA2T3",
  "term_id": "GO:0003714"
}